{
  "gene_name": "Zinc finger protein 239",
  "term_label": "Unknown cellular component",
  "gene": "UniProtKB:Q16600",
  "gene_symbol": "ZNF239",
  "term_id": "UNKNOWN:0003"
}